{
  "gene_symbol": "NUP98",
  "gene": "UniProtKB:P52948",
  "term_id": "GO:0034398",
  "term_label": "telomere tethering at nuclear periphery",
  "gene_name": "Nuclear pore complex protein Nup98-Nup96"
}